{
  "gene_symbol": "NANOS1",
  "gene_name": "Nanos homolog 1",
  "gene": "UniProtKB:Q8WY41",
  "term_label": "mRNA binding",
  "term_id": "GO:0003729"
}